{
  "gene": "UniProtKB:Q6ZN08",
  "gene_name": "Putative zinc finger protein 66",
  "gene_symbol": "ZNF66",
  "term_label": "regulation of DNA-templated transcription",
  "term_id": "GO:0006355"
}